{
  "gene_symbol": "A4GALT",
  "term_label": "galactosyltransferase activity",
  "gene_name": "Lactosylceramide 4-alpha-galactosyltransferase",
  "term_id": "GO:0008378",
  "gene": "UniProtKB:Q9NPC4"
}